{
  "term_id": "GO:0004693",
  "gene": "UniProtKB:Q00534",
  "gene_symbol": "CDK6",
  "term_label": "cyclin-dependent protein serine/threonine kinase activity",
  "gene_name": "Cyclin-dependent kinase 6"
}